{
  "term_label": "Unknown molecular function",
  "gene": "UniProtKB:Q9NUR3",
  "gene_symbol": "TMEM74B",
  "gene_name": "Transmembrane protein 74B",
  "term_id": "UNKNOWN:0001"
}